{
  "gene_name": "Putative uncharacterized protein FLJ44553",
  "term_id": "UNKNOWN:0003",
  "term_label": "Unknown cellular component",
  "gene": "UniProtKB:Q86TA4",
  "gene_symbol": "Q86TA4"
}